{
  "term_label": "guanyl-nucleotide exchange factor activity",
  "gene": "UniProtKB:Q9UKW4",
  "term_id": "GO:0005085",
  "gene_name": "Guanine nucleotide exchange factor VAV3",
  "gene_symbol": "VAV3"
}